{
  "gene_symbol": "OSTC",
  "term_id": "GO:0008250",
  "gene_name": "Oligosaccharyltransferase complex subunit OSTC",
  "term_label": "oligosaccharyltransferase complex",
  "gene": "UniProtKB:Q9NRP0"
}